pyrroloquinoline quinone biosynthetic process [GO:0018189] (biological process) References: PMID:7665488 Sources: RESID:AA0283 Also known as: PQQ biosynthesis, PQQ biosynthetic process, coenzyme pyrroloquinoline-quinone biosynthesis, coenzyme pyrroloquinoline-quinone biosynthetic process, pyrroloquinoline quinone anabolism, pyrroloquinoline quinone biosynthesis, pyrroloquinoline quinone formation, pyrroloquinoline quinone synthesis, pyrroloquinoline-quinone biosynthesis, pyrroloquinoline-quinone biosynthetic process Definition: The chemical reactions and pathways resulting in the formation of the cofactor pyrroloquinoline quinone (PQQ); it is synthesized from a small peptide containing tyrosine and glutamic acid; these amino acids in the peptide are multiply cross-linked and the rest of the peptide is removed. Relationships: is a type of ketone biosynthetic process [GO:0042181]; is a type of tricarboxylic acid biosynthetic process [GO:0072351]